{
  "term_id": "GO:0043161",
  "gene_name": "AN1-type zinc finger protein 2B",
  "term_label": "proteasome-mediated ubiquitin-dependent protein catabolic process",
  "gene": "UniProtKB:Q8WV99",
  "gene_symbol": "ZFAND2B"
}